{
  "gene_name": "Serine_threonine-protein kinase DCLK2",
  "gene_symbol": "DCLK2",
  "gene": "UniProtKB:Q8N568",
  "term_id": "GO:0004674",
  "term_label": "protein serine/threonine kinase activity"
}